{
  "gene_name": "CREB3 regulatory factor",
  "gene": "UniProtKB:Q8IUR6",
  "gene_symbol": "CREBRF",
  "term_id": "GO:0000981",
  "term_label": "DNA-binding transcription factor activity, RNA polymerase II-specific"
}